{
  "term_label": "chemokine activity",
  "gene": "UniProtKB:P02776",
  "gene_name": "Platelet factor 4",
  "gene_symbol": "PF4",
  "term_id": "GO:0008009"
}